{
  "term_label": "positive regulation of cytosolic calcium ion concentration",
  "term_id": "GO:0007204",
  "gene_name": "Chemokine XC receptor 1",
  "gene": "UniProtKB:P46094",
  "gene_symbol": "XCR1"
}